{
  "gene_symbol": "RASL11A",
  "gene_name": "Ras-like protein family member 11A",
  "term_id": "UNKNOWN:0002",
  "gene": "UniProtKB:Q6T310",
  "term_label": "Unknown biological process"
}